{
  "term_label": "plasma membrane",
  "term_id": "GO:0005886",
  "gene": "UniProtKB:P04435",
  "gene_name": "T cell receptor beta variable 7-9",
  "gene_symbol": "TRBV7-9"
}